{
  "gene": "UniProtKB:Q156A1",
  "term_label": "Unknown biological process",
  "gene_symbol": "ATXN8",
  "gene_name": "Ataxin-8",
  "term_id": "UNKNOWN:0002"
}